{
  "term_id": "GO:0016035",
  "gene_symbol": "MAD2L2",
  "gene_name": "Mitotic spindle assembly checkpoint protein MAD2B",
  "gene": "UniProtKB:Q9UI95",
  "term_label": "zeta DNA polymerase complex"
}